{
  "term_label": "dorsal/ventral pattern formation",
  "gene_symbol": "TLL2",
  "gene_name": "Tolloid-like protein 2",
  "term_id": "GO:0009953",
  "gene": "UniProtKB:Q9Y6L7"
}